{
  "term_label": "excitatory postsynaptic potential",
  "gene_name": "Glutamate receptor ionotropic, NMDA 2C",
  "gene": "UniProtKB:Q14957",
  "gene_symbol": "GRIN2C",
  "term_id": "GO:0060079"
}